{
  "gene": "UniProtKB:Q9GZT9",
  "gene_symbol": "EGLN1",
  "gene_name": "Egl nine homolog 1",
  "term_label": "ferrous iron binding",
  "term_id": "GO:0008198"
}